{
  "term_id": "GO:0034446",
  "gene_symbol": "LAMC1",
  "gene_name": "Laminin subunit gamma-1",
  "term_label": "substrate adhesion-dependent cell spreading",
  "gene": "UniProtKB:P11047"
}